{
  "gene": "UniProtKB:O60229",
  "term_label": "intracellular signal transduction",
  "gene_name": "Kalirin",
  "gene_symbol": "KALRN",
  "term_id": "GO:0035556"
}